behavioral response to ethanol [GO:0048149] (biological process) Also known as: behavioural response to ethanol Definition: Any process that results in a change in the behavior of an organism as a result of an ethanol stimulus. Relationships: is a type of adult behavior [GO:0030534]; is part of response to ethanol [GO:0045471] Sources: GOC:jid